{
  "term_label": "membrane",
  "term_id": "GO:0016020",
  "gene_name": "Myotubularin-related protein 12",
  "gene": "UniProtKB:Q9C0I1",
  "gene_symbol": "MTMR12"
}